{
  "term_id": "UNKNOWN:0003",
  "gene": "UniProtKB:Q3MIV0",
  "term_label": "Unknown cellular component",
  "gene_symbol": "KRTAP22-1",
  "gene_name": "Keratin-associated protein 22-1"
}